axonogenesis [GO:0007409] (BP) Note: Note that 'axonogenesis' differs from 'axon development' in that the latter also covers other processes, such as axon regeneration (regrowth after loss or damage, not necessarily of the whole axon). Sources: GOC:dph, GOC:jid, GOC:pg, GOC:pr, ISBN:0198506732 Subtypes: central nervous system neuron axonogenesis [GO:0021955], GO:0048936, GO:0060385, axon arborization [GO:0140060] Definition: De novo generation of a long process of a neuron, including the terminal branched region. Refers to the morphogenesis or creation of shape or form of the developing axon, which carries efferent (outgoing) action potentials from the cell body towards target cells. Also known as: axon morphogenesis, neuron long process generation, axon growth Relationships: is a type of GO:0048812; is part of cell morphogenesis involved in neuron differentiation [GO:0048667]; is part of axon development [GO:0061564] Regulation: regulated by GO:0050770; negatively regulated by GO:0050771; positively regulated by GO:0050772